{
  "term_id": "GO:0008441",
  "gene_symbol": "BPNT1",
  "gene_name": "3'(2'),5'-bisphosphate nucleotidase 1",
  "gene": "UniProtKB:O95861",
  "term_label": "3'(2'),5'-bisphosphate nucleotidase activity"
}